{
  "gene": "UniProtKB:A0A1W2PQ09",
  "term_label": "RNA polymerase II preinitiation complex assembly",
  "term_id": "GO:0051123",
  "gene_name": "TATA-box-binding protein-associated factor 11-like protein 11",
  "gene_symbol": "TAF11L11"
}